{
  "gene": "UniProtKB:Q9NXX6",
  "term_label": "Smc5-Smc6 complex",
  "gene_name": "Non-structural maintenance of chromosomes element 4 homolog A",
  "gene_symbol": "NSMCE4A",
  "term_id": "GO:0030915"
}